{
  "term_id": "GO:0006357",
  "gene": "UniProtKB:Q8N8Y5",
  "term_label": "regulation of transcription by RNA polymerase II",
  "gene_name": "Zinc finger protein 41 homolog",
  "gene_symbol": "ZFP41"
}